{
  "gene_name": "Mediator of RNA polymerase II transcription subunit 28",
  "gene": "UniProtKB:Q9H204",
  "gene_symbol": "MED28",
  "term_id": "UNKNOWN:0001",
  "term_label": "Unknown molecular function"
}